{
  "gene_symbol": "SMAD5",
  "term_id": "GO:0000981",
  "term_label": "DNA-binding transcription factor activity, RNA polymerase II-specific",
  "gene": "UniProtKB:Q99717",
  "gene_name": "Mothers against decapentaplegic homolog 5"
}